cellular response to 3-methylcholanthrene [GO:1904682] (biological process) Relationships: is a type of cellular response to polycyclic arene [GO:1903166]; is a type of response to 3-methylcholanthrene [GO:1904681] References: PMID:9224771 Sources: GOC:TermGenie, GOC:mr, GO_REF:0000071 Definition: Any process that results in a change in state or activity of a cell (in terms of movement, secretion, enzyme production, gene expression, etc.) as a result of a 3-methylcholanthrene stimulus.